cellular response to oxidative stress [GO:0034599] (biological process) Sources: GOC:mah Subtypes: cellular response to reactive oxygen species [GO:0034614], symbiont defense to host-produced reactive oxygen species [GO:0052164], cellular response to hydroperoxide [GO:0071447] Definition: Any process that results in a change in state or activity of a cell (in terms of movement, secretion, enzyme production, gene expression, etc.) as a result of oxidative stress, a state often resulting from exposure to high levels of reactive oxygen species, e.g. superoxide anions, hydrogen peroxide (H2O2), and hydroxyl radicals. Also known as: adaptive response to oxidative stress Relationships: is a type of GO:0006979; is a type of cellular response to chemical stress [GO:0062197] Regulation: regulated by GO:1900407; negatively regulated by GO:1900408; positively regulated by GO:1900409